{
  "gene": "UniProtKB:Q6P4D5",
  "gene_name": "PABIR family member 1",
  "term_id": "GO:0005634",
  "term_label": "nucleus",
  "gene_symbol": "PABIR3"
}